{
  "gene_symbol": "ASIC5",
  "gene": "UniProtKB:Q9NY37",
  "term_label": "ligand-gated sodium channel activity",
  "term_id": "GO:0015280",
  "gene_name": "Acid-sensing ion channel 5"
}